regulation of hypoxanthine transport [GO:0035345] (biological process) Definition: Any process that modulates the frequency, rate or extent of the directed movement of hypoxanthine into, out of or within a cell, or between cells, by means of some agent such as a transporter or pore. Relationships: is a type of regulation of nucleobase-containing compound transport [GO:0032239]; regulates GO:0035344 Also known as: regulation of 6-hydroxypurine transport Subtypes: positive regulation of hypoxanthine transport [GO:0035346], negative regulation of hypoxanthine transport [GO:0035347] Sources: GOC:bf